{
  "gene_name": "Serine_threonine-protein kinase PLK4",
  "gene": "UniProtKB:O00444",
  "term_id": "GO:0005634",
  "term_label": "nucleus",
  "gene_symbol": "PLK4"
}